{
  "gene_name": "Protein DBF4 homolog A",
  "gene_symbol": "DBF4",
  "gene": "UniProtKB:Q9UBU7",
  "term_id": "GO:0043539",
  "term_label": "protein serine/threonine kinase activator activity"
}